intercellular bridge organization [GO:0043063] (biological process) Relationships: is a type of extracellular structure organization [GO:0043062] Sources: GOC:jid Definition: A process that is carried out at the cellular level which results in the assembly, arrangement of constituent parts, or disassembly of the intracellular bridge. An intracellular bridge is a direct link between the cytoplasms of sister cells that allows cells to communicate with one another. Also known as: intercellular bridge organisation, intercellular bridge organization and biogenesis Subtypes: germline ring canal formation [GO:0030725]